chitin metabolic process [GO:0006030] (biological process) Also known as: beta-1,4-linked N-acetylglucosamine metabolic process, beta-1,4-linked N-acetylglucosamine metabolism, chitin metabolism Definition: The chemical reactions and pathways involving chitin, a linear polysaccharide consisting of beta-(1->4)-linked N-acetyl-D-glucosamine residues. Relationships: is a type of aminoglycan metabolic process [GO:0006022]; is a type of amino sugar metabolic process [GO:0006040] Sources: GOC:jl, ISBN:0198506732 Regulation: RO_0002211 by regulation of chitin metabolic process [GO:0032882] Subtypes: GO:0006031, chitin catabolic process [GO:0006032]